response to cyclophosphamide [GO:1902518] (biological process) Definition: Any process that results in a change in state or activity of a cell or an organism (in terms of movement, secretion, enzyme production, gene expression, etc.) as a result of a cyclophosphamide stimulus. References: PMID:23648065 Sources: GOC:TermGenie, GOC:dw Relationships: is a type of GO:1901698 Note: Note that this term is in the subset of terms that should not be used for direct manual annotation of gene products. It was created to be used for cross-referencing by other ontologies. Direct annotations to this term may be amended during annotation QC.